EGAD pathway [GO:0140624] (biological process) References: PMID:31368600 Definition: The protein catabolic pathway which selectively extracts ER-resident membrane proteins exported to the Golgi and endosomes for degradation by cytosolic proteasomes. It begins with phosphorylation of the ER-resident membrane protein, which triggers export of the protein from the ER to the Golgi and endosomes, followed by polyubiquitination by the Dsc E3 ubiquitin ligase complex and extraction of the ubiquitinated target, and ends with proteasomal degradation. Relationships: is a type of proteasomal protein catabolic process [GO:0010498]